{
  "gene": "UniProtKB:Q9NVA2",
  "gene_symbol": "SEPTIN11",
  "term_label": "cell division site",
  "term_id": "GO:0032153",
  "gene_name": "Septin-11"
}